benzoic acid glucosyltransferase activity [GO:0052641] (molecular function) Sources: MetaCyc:RXN-11660 Definition: Catalysis of the reaction: benzoic acid + UDP-glucose = benzoic acid glucose ester + UDP. Relationships: is a type of UDP-glucosyltransferase activity [GO:0035251] Also known as: UDP:glucose:BA glucosyltransferase activity, UDP:glucose:benzoate glucosyltransferase activity, UDP:glucose:benzoic acid glucosyltransferase activity, benzoate glucosyltransferase activity